metanephros development [GO:0001656] (biological process) Subtypes: regulation of metanephric glomerulus development [GO:0072298] Regulation: RO_0002211 by regulation of metanephros development [GO:0072215]; positively regulated by positive regulation of metanephros development [GO:0072216]; RO_0002212 by GO:0072217 Definition: The process whose specific outcome is the progression of the metanephros over time, from its formation to the mature structure. In mammals, the metanephros is the excretory organ of the fetus, which develops into the mature kidney and is formed from the rear portion of the nephrogenic cord. The metanephros is an endocrine and metabolic organ that filters the blood and excretes the end products of body metabolism in the form of urine. Relationships: is a type of GO:0001822 Sources: GOC:bf, ISBN:0192800752